{
  "term_id": "GO:0007214",
  "term_label": "gamma-aminobutyric acid signaling pathway",
  "gene": "UniProtKB:P04899",
  "gene_name": "Guanine nucleotide-binding protein G(i) subunit alpha-2",
  "gene_symbol": "GNAI2"
}